{
  "term_id": "GO:0005886",
  "gene": "UniProtKB:P0C604",
  "term_label": "plasma membrane",
  "gene_name": "Olfactory receptor 4A8",
  "gene_symbol": "OR4A8"
}